{
  "gene": "UniProtKB:O60422",
  "gene_name": "One cut domain family member 3",
  "term_id": "GO:0000978",
  "term_label": "RNA polymerase II cis-regulatory region sequence-specific DNA binding",
  "gene_symbol": "ONECUT3"
}